{
  "term_id": "UNKNOWN:0002",
  "gene_name": "Elastin",
  "term_label": "Unknown biological process",
  "gene_symbol": "ELN",
  "gene": "UniProtKB:P15502"
}